{
  "gene": "UniProtKB:Q8N831",
  "term_label": "Unknown biological process",
  "term_id": "UNKNOWN:0002",
  "gene_name": "Testis-specific Y-encoded-like protein 6",
  "gene_symbol": "TSPYL6"
}